{
  "gene_symbol": "PEX5L",
  "term_label": "peroxisomal membrane",
  "term_id": "GO:0005778",
  "gene": "UniProtKB:Q8IYB4",
  "gene_name": "PEX5-related protein"
}